{
  "term_id": "UNKNOWN:0001",
  "gene_symbol": "LRRC2",
  "gene_name": "Leucine-rich repeat-containing protein 2",
  "gene": "UniProtKB:Q9BYS8",
  "term_label": "Unknown molecular function"
}